{
  "term_label": "Unknown cellular component",
  "gene_name": "TP53-target gene 3 protein",
  "gene_symbol": "TP53TG3F",
  "gene": "UniProtKB:Q9ULZ0",
  "term_id": "UNKNOWN:0003"
}